{
  "gene_symbol": "SMCO1",
  "term_label": "Unknown cellular component",
  "gene_name": "Single-pass membrane and coiled-coil domain-containing protein 1",
  "gene": "UniProtKB:Q147U7",
  "term_id": "UNKNOWN:0003"
}